{
  "gene_name": "DNA dC-dU-editing enzyme APOBEC-3D",
  "gene": "UniProtKB:Q96AK3",
  "gene_symbol": "APOBEC3D",
  "term_id": "GO:0051607",
  "term_label": "defense response to virus"
}